{
  "term_id": "GO:0005634",
  "gene": "UniProtKB:Q96RU7",
  "gene_symbol": "TRIB3",
  "term_label": "nucleus",
  "gene_name": "Tribbles homolog 3"
}